{
  "gene_name": "Tumor necrosis factor receptor superfamily member 13C",
  "gene": "UniProtKB:Q96RJ3",
  "gene_symbol": "TNFRSF13C",
  "term_label": "B cell costimulation",
  "term_id": "GO:0031296"
}